{
  "gene": "UniProtKB:Q9BYT5",
  "gene_symbol": "KRTAP2-2",
  "term_label": "Unknown biological process",
  "gene_name": "Keratin-associated protein 2-2",
  "term_id": "UNKNOWN:0002"
}